positive regulation of non-canonical Wnt signaling pathway [GO:2000052] (biological process) Definition: Any process that activates or increases the frequency, rate or extent of non-canonical Wnt-activated signaling pathway. Sources: GOC:obol, GOC:yaf Subtypes: positive regulation of Wnt signaling pathway, calcium modulating pathway [GO:0045813], positive regulation of Frizzled Nuclear Import pathway [GO:0140711], positive regulation of Wnt signaling pathway, planar cell polarity pathway [GO:2000096] Also known as: positive regulation of beta-catenin-independent Wnt receptor signaling pathway, positive regulation of non-canonical Wnt receptor signaling pathway, positive regulation of non-canonical Wnt receptor signalling pathway, positive regulation of non-canonical Wnt-activated signaling pathway Relationships: is a type of positive regulation of Wnt signaling pathway [GO:0030177]; is_a regulation of non-canonical Wnt signaling pathway [GO:2000050]; positively regulates non-canonical Wnt signaling pathway [GO:0035567]